{
  "gene_name": "Protein WFDC11",
  "term_id": "GO:0019731",
  "gene_symbol": "WFDC11",
  "term_label": "antibacterial humoral response",
  "gene": "UniProtKB:Q8NEX6"
}